{
  "term_id": "UNKNOWN:0002",
  "gene_name": "Serine hydrolase-like protein",
  "gene": "UniProtKB:Q9NQF3",
  "term_label": "Unknown biological process",
  "gene_symbol": "SERHL"
}